18S rRNA cytidine N-acetyltransferase activity [GO:1990883] (molecular function) Relationships: is a type of N-acetyltransferase activity [GO:0008080] References: PMID:25402480 Sources: RHEA:51424 Definition: Catalysis of the reaction: a cytidine in 18S rRNA + acetyl-CoA + ATP + H2O = an N(4)-acetylcytidine in 18S rRNA + ADP + phosphate + CoA + H+.